{
  "gene": "UniProtKB:Q6ZUB1",
  "gene_name": "Spermatogenesis-associated protein 31E1",
  "gene_symbol": "SPATA31E1",
  "term_label": "Unknown cellular component",
  "term_id": "UNKNOWN:0003"
}